regulation of amyloid fibril formation [GO:1905906] (biological process) Subtypes: negative regulation of amyloid fibril formation [GO:1905907], GO:1905908 Relationships: is_a regulation of protein metabolic process [GO:0051246]; is_a regulation of supramolecular fiber organization [GO:1902903]; regulates GO:1990000 Definition: Any process that modulates the frequency, rate or extent of amyloid fibril formation. Also known as: regulation of amyloid fibril assembly, regulation of amyloid structure assembly, regulation of amyloid structure formation References: PMID:23106396 Sources: GOC:TermGenie, GOC:aruk, GOC:bc, GO_REF:0000058 Note: Although deposition of amyloid fibrils is associated with diseases, e.g. Alzheimer's disease, amyloid formation is a normal process. Disease occurs when the balance between amyloid formation and clearance is disrupted (reviewed e.g. in PMID:29654159 and PMID:28937655). An example of a normal amyloid complex is composed of human RIP1 and RIP3 kinases (PMID:22817896).